apical constriction involved in gastrulation [GO:0003384] (biological process) Definition: The actin-mediated process that results in the contraction of the apical end of a polarized columnar epithelial cell, contributing to the process of gastrulation. Sources: GOC:ascb_2009, GOC:dph, GOC:tb Relationships: is a type of apical constriction [GO:0003383]; is part of epithelial cell morphogenesis involved in gastrulation [GO:0003381] Subtypes: apical constriction involved in ventral furrow formation [GO:0110072]